{
  "gene_symbol": "CNGB1",
  "term_label": "photoreceptor outer segment",
  "term_id": "GO:0001750",
  "gene": "UniProtKB:Q14028",
  "gene_name": "Cyclic nucleotide-gated cation channel beta-1"
}